potassium ion transmembrane transport [GO:0071805] (BP) Sources: GOC:mah Definition: A process in which a potassium ion is transported from one side of a membrane to the other. Subtypes: potassium ion export across plasma membrane [GO:0097623], GO:0140141, GO:1990573 Regulation: regulated by regulation of potassium ion transmembrane transport [GO:1901379]; negatively regulated by negative regulation of potassium ion transmembrane transport [GO:1901380]; positively regulated by positive regulation of potassium ion transmembrane transport [GO:1901381] Also known as: potassium ion membrane transport, high affinity potassium ion import, high affinity potassium ion uptake, high-affinity potassium ion import, high-affinity potassium ion uptake Relationships: is a type of potassium ion transport [GO:0006813]; is a type of monoatomic cation transmembrane transport [GO:0098655] Note: Note that this term is not intended for use in annotating lateral movement within membranes.